{
  "term_label": "mRNA binding",
  "gene_name": "Putative RNA-binding protein Luc7-like 2",
  "term_id": "GO:0003729",
  "gene_symbol": "LUC7L2",
  "gene": "UniProtKB:Q9Y383"
}